negative regulation of cyclodextrin catabolic process [GO:2000958] (BP) Relationships: is a type of negative regulation of catabolic process [GO:0009895]; is a type of negative regulation of macromolecule metabolic process [GO:0010605]; is a type of GO:0045912; is a type of regulation of cyclodextrin catabolic process [GO:2000957]; negatively regulates GO:2000901 Also known as: negative regulation of cyclodextrin catabolism Sources: GOC:mengo_curators Definition: Any process that stops, prevents or reduces the frequency, rate or extent of cyclodextrin catabolic process.